{
  "term_label": "regulation of alternative mRNA splicing, via spliceosome",
  "gene": "UniProtKB:Q13242",
  "gene_name": "Serine_arginine-rich splicing factor 9",
  "term_id": "GO:0000381",
  "gene_symbol": "SRSF9"
}